aminoglycoside phosphotransferase activity [GO:0034071] (MF) Definition: Catalysis of the reaction: ATP + aminoglycoside = ADP + phosphoaminoglycoside. Sources: GOC:cb, GOC:mah Also known as: aminoglycoside kinase activity Relationships: is a type of kinase activity [GO:0016301]; is a type of phosphotransferase activity, alcohol group as acceptor [GO:0016773] Subtypes: hygromycin-B 7''-O-phosphotransferase activity [GO:0008904], kanamycin kinase activity [GO:0008910], GO:0047333, streptomycin 3''-kinase activity [GO:0050299], aminoglycoside 6-kinase activity [GO:0050300]